zinc ion export from vacuole [GO:0140147] (biological process) Sources: GOC:vw, PMC:PMC203372 Definition: The directed movement of zinc ions from inside the vacuole across the vacuolar membrane and into the cytosol. Relationships: is a type of GO:0034486; is a type of zinc ion transmembrane transport [GO:0071577]